{
  "gene_symbol": "BCLAF1",
  "term_label": "mediator complex",
  "gene_name": "Bcl-2-associated transcription factor 1",
  "term_id": "GO:0016592",
  "gene": "UniProtKB:Q9NYF8"
}